{
  "gene": "UniProtKB:Q9P0J7",
  "term_label": "Unknown molecular function",
  "gene_name": "E3 ubiquitin-protein ligase KCMF1",
  "term_id": "UNKNOWN:0001",
  "gene_symbol": "KCMF1"
}